{
  "gene": "UniProtKB:O60238",
  "gene_name": "BCL2_adenovirus E1B 19 kDa protein-interacting protein 3-like",
  "term_id": "GO:0005635",
  "term_label": "nuclear envelope",
  "gene_symbol": "BNIP3L"
}